regulation of ER to Golgi vesicle-mediated transport [GO:0060628] (biological process) Sources: GOC:dph, GOC:tb Relationships: is a type of GO:0032386; is a type of regulation of vesicle-mediated transport [GO:0060627]; regulates endoplasmic reticulum to Golgi vesicle-mediated transport [GO:0006888] Definition: Any process that modulates the rate, frequency, or extent of ER to Golgi vesicle-mediated transport, the directed movement of substances from the endoplasmic reticulum (ER) to the Golgi, mediated by COP II vesicles. Small COP II coated vesicles form from the ER and then fuse directly with the cis-Golgi. Larger structures are transported along microtubules to the cis-Golgi. Subtypes: GO:1902953